dopamine metabolic process [GO:0042417] (biological process) Regulation: regulated by regulation of dopamine metabolic process [GO:0042053]; negatively regulated by GO:0045963; positively regulated by positive regulation of dopamine metabolic process [GO:0045964] Subtypes: dopamine biosynthetic process [GO:0042416], GO:0042420 Relationships: is a type of catecholamine metabolic process [GO:0006584] Definition: The chemical reactions and pathways involving dopamine, a catecholamine neurotransmitter and a metabolic precursor of noradrenaline and adrenaline. Also known as: dopamine metabolism Sources: GOC:jl, ISBN:0198506732